{
  "term_label": "leukocyte cell-cell adhesion",
  "gene": "UniProtKB:P57087",
  "term_id": "GO:0007159",
  "gene_symbol": "JAM2",
  "gene_name": "Junctional adhesion molecule B"
}